{
  "gene": "UniProtKB:Q8TEK3",
  "gene_symbol": "DOT1L",
  "term_label": "nucleus",
  "gene_name": "Histone-lysine N-methyltransferase, H3 lysine-79 specific",
  "term_id": "GO:0005634"
}